{
  "term_label": "Unknown molecular function",
  "gene": "UniProtKB:Q9Y2V7",
  "gene_symbol": "COG6",
  "gene_name": "Conserved oligomeric Golgi complex subunit 6",
  "term_id": "UNKNOWN:0001"
}